{
  "term_label": "transcription cis-regulatory region binding",
  "gene_symbol": "ZNF493",
  "gene_name": "Zinc finger protein 493",
  "term_id": "GO:0000976",
  "gene": "UniProtKB:Q6ZR52"
}